heparin-sulfate lyase activity [GO:0015021] (molecular function) Definition: Catalysis of the elimination of sulfate; appears to act on linkages between N-acetyl-D-glucosamine and uronate. Product is an unsaturated sugar. Relationships: is a type of carbon-oxygen lyase activity, acting on polysaccharides [GO:0016837] Sources: EC:4.2.2.8 Also known as: heparin-sulphate lyase activity, heparitin-sulfate lyase activity, [heparan sulfate]-sulfate lyase activity, heparin-sulfate eliminase activity, heparitinase I, heparitinase II